regulation of glial cell-derived neurotrophic factor receptor signaling pathway involved in ureteric bud formation [GO:2000733] (biological process) Subtypes: GO:2000734, positive regulation of glial cell-derived neurotrophic factor receptor signaling pathway involved in ureteric bud formation [GO:2000735] Also known as: regulation of GDNF receptor signaling pathway of ureteric bud formation, regulation of glial cell derived neurotrophic factor receptor signaling pathway of ureteric bud formation, regulation of glial cell line-derived neurotrophic factor receptor signalling pathway of ureteric bud formation, regulation of glial cell-derived neurotrophic factor receptor signaling pathway of ureteric bud formation, regulation of glial cell-derived neurotrophic factor receptor signalling pathway of ureteric bud formation Sources: GOC:obol Relationships: is a type of regulation of signal transduction [GO:0009966]; regulates glial cell-derived neurotrophic factor receptor signaling pathway involved in ureteric bud formation [GO:2000701] Definition: Any process that modulates the frequency, rate or extent of glial cell-derived neurotrophic factor receptor signaling pathway involved in ureteric bud formation.